{
  "gene_symbol": "IFITM5",
  "term_id": "GO:0005886",
  "gene": "UniProtKB:A6NNB3",
  "gene_name": "Interferon-induced transmembrane protein 5",
  "term_label": "plasma membrane"
}